{
  "gene": "UniProtKB:Q8NFQ5",
  "term_id": "UNKNOWN:0002",
  "term_label": "Unknown biological process",
  "gene_name": "BPI fold-containing family B member 6",
  "gene_symbol": "BPIFB6"
}